{
  "gene_symbol": "GPSM1",
  "term_id": "UNKNOWN:0003",
  "gene": "UniProtKB:Q86YR5",
  "term_label": "Unknown cellular component",
  "gene_name": "G-protein-signaling modulator 1"
}